{
  "gene_name": "Cilia- and flagella-associated protein 100",
  "term_label": "Unknown molecular function",
  "gene_symbol": "CFAP100",
  "term_id": "UNKNOWN:0001",
  "gene": "UniProtKB:Q494V2"
}